histone H3K37 methyltransferase activity [GO:0062122] (molecular function) Note: Comment: Note that the residue position corresponds to the canonical human H3 histone (UniProtKB:P84243); this residue is conserved across all eukaryotes. Residue 1 is the first residue following removal of the initiating Methionine (Met). Note that each histone is encoded by multiple genes, and sequences may vary across different genes within an organism. Also known as: histone H3K37 methylase activity, histone lysine N-methyltransferase activity (H3-K37 specific), histone methyltransferase activity (H3-K37 specific), histone-H3K37 methyltransferase activity References: PMID:30773398 Definition: Catalysis of the reaction: S-adenosyl-L-methionine + histone H3 L-lysine (position 37) = S-adenosyl-L-homocysteine + histone H3 N6-methyl-L-lysine (position 37). This reaction is the addition of a methyl group to the lysine residue at position 37 of the histone H3 protein. Relationships: is a type of protein-lysine N-methyltransferase activity [GO:0016279]; is a type of histone H3 methyltransferase activity [GO:0140938]